{
  "gene": "UniProtKB:Q5T0L3",
  "term_label": "Unknown molecular function",
  "gene_name": "Spermatogenesis-associated protein 46",
  "term_id": "UNKNOWN:0001",
  "gene_symbol": "SPATA46"
}